positive regulation of smooth muscle cell differentiation [GO:0051152] (biological process) Subtypes: GO:1905065, GO:2000063, positive regulation of kidney smooth muscle cell differentiation [GO:2000358] Also known as: up regulation of smooth muscle cell differentiation, up-regulation of smooth muscle cell differentiation, upregulation of smooth muscle cell differentiation, activation of smooth muscle cell differentiation, stimulation of smooth muscle cell differentiation Relationships: is a type of positive regulation of muscle cell differentiation [GO:0051149]; is a type of regulation of smooth muscle cell differentiation [GO:0051150]; RO_0002213 smooth muscle cell differentiation [GO:0051145] Definition: Any process that activates or increases the frequency, rate or extent of smooth muscle cell differentiation. Sources: CL:0000192, GOC:ai